regulation of interleukin-4-mediated signaling pathway [GO:1902214] (biological process) Definition: Any process that modulates the frequency, rate or extent of interleukin-4-mediated signaling pathway. Also known as: regulation of IL-4-mediated signaling pathway, regulation of interleukin-4-mediated signalling pathway References: PMID:17210636 Sources: GOC:TermGenie Subtypes: negative regulation of interleukin-4-mediated signaling pathway [GO:1902215], positive regulation of interleukin-4-mediated signaling pathway [GO:1902216] Relationships: is a type of regulation of cytokine-mediated signaling pathway [GO:0001959]; regulates interleukin-4-mediated signaling pathway [GO:0035771]